ERBB2-EGFR signaling pathway [GO:0038134] (biological process) Relationships: is a type of epidermal growth factor receptor signaling pathway [GO:0007173]; is a type of GO:0038128 References: PMID:16460914 Sources: GOC:signaling Also known as: EGFR-HER2 signaling pathway, ERBB2-EGFR signalling pathway Definition: The series of molecular signals initiated by binding of a ligand to an epidermal growth factor receptor (EGFR/ERBB1) on the surface of a cell, followed by transmission of the signal by a heterodimeric complex of ERBB2 and EGFR. ERBB2, which does not bind any known ligand, is activated through formation of a heterodimer with another ligand-activated ERBB family member such as EGFR.